{
  "term_id": "GO:0005886",
  "gene_name": "Olfactory receptor 2F1",
  "gene": "UniProtKB:Q13607",
  "gene_symbol": "OR2F1",
  "term_label": "plasma membrane"
}